P2Y11 nucleotide receptor binding [GO:0031820] (MF) Also known as: P2Y11 nucleotide receptor ligand Definition: Binding to a P2Y11 nucleotide receptor. Relationships: is_a G protein-coupled nucleotide receptor binding [GO:0031811] Sources: GOC:mah, GOC:nln